{
  "gene_symbol": "FIZ1",
  "gene": "UniProtKB:Q96SL8",
  "term_id": "UNKNOWN:0003",
  "gene_name": "Flt3-interacting zinc finger protein 1",
  "term_label": "Unknown cellular component"
}